{
  "term_label": "negative regulation of transcription by RNA polymerase II",
  "gene_symbol": "HEY2",
  "gene": "UniProtKB:Q9UBP5",
  "term_id": "GO:0000122",
  "gene_name": "Hairy_enhancer-of-split related with YRPW motif protein 2"
}